{
  "gene": "UniProtKB:Q1MSJ5",
  "gene_name": "Centrosome and spindle pole-associated protein 1",
  "term_label": "spindle pole",
  "gene_symbol": "CSPP1",
  "term_id": "GO:0000922"
}